glucosinolate transport [GO:1901349] (biological process) Relationships: is a type of nitrogen compound transport [GO:0071705]; is a type of sulfur compound transport [GO:0072348]; is_a carbohydrate derivative transport [GO:1901264] Sources: GOC:TermGenie Definition: The directed movement of a glucosinolate into, out of or within a cell, or between cells, by means of some agent such as a transporter or pore. Subtypes: phloem glucosinolate loading [GO:0090449]